{
  "gene_symbol": "OR5C1",
  "gene": "UniProtKB:Q8NGR4",
  "term_id": "GO:0004984",
  "gene_name": "Olfactory receptor 5C1",
  "term_label": "olfactory receptor activity"
}